{
  "term_id": "GO:0042288",
  "term_label": "MHC class I protein binding",
  "gene_name": "Paired immunoglobulin-like type 2 receptor alpha",
  "gene_symbol": "PILRA",
  "gene": "UniProtKB:Q9UKJ1"
}